teichuronic acid biosynthetic process [GO:0050845] (biological process) Definition: The chemical reactions and pathways resulting in the formation of teichuronic acid, a polymer containing chains of uronic acids and N-acetylglucosamine found in the cell wall, membrane or capsule of Gram-positive bacteria. Sources: ISBN:0815108893 Also known as: teichuronic acid anabolism, teichuronic acid biosynthesis, teichuronic acid formation, teichuronic acid synthesis Relationships: is a type of GO:0016053; is a type of cell wall macromolecule biosynthetic process [GO:0044038]; is part of peptidoglycan-based cell wall biogenesis [GO:0009273]